{
  "gene": "UniProtKB:P0C7V8",
  "term_id": "UNKNOWN:0001",
  "gene_name": "DDB1- and CUL4-associated factor 8-like protein 2",
  "term_label": "Unknown molecular function",
  "gene_symbol": "DCAF8L2"
}